spinal cord dorsal/ventral patterning [GO:0021513] (biological process) Definition: The process that regulates the coordinated growth and differentiation that establishes the non-random dorsal-ventral spatial arrangement of the spinal cord. Sources: GOC:cls, GOC:dgh, GOC:dph, GOC:jid, GO_REF:0000021 Also known as: spinal cord dorsal-ventral patterning, spinal cord dorsoventral patterning Relationships: is a type of dorsal/ventral pattern formation [GO:0009953]; is part of spinal cord patterning [GO:0021511]